steroid 15-alpha-hydroxylase activity [GO:0008388] (molecular function) Also known as: cytochrome P450 CYP2A4 References: PMID:2703500 Sources: RHEA:83179 Relationships: is a type of steroid hydroxylase activity [GO:0008395]; is a type of oxidoreductase activity, acting on paired donors, with incorporation or reduction of molecular oxygen [GO:0016705] Definition: Catalysis of the reaction: reduced [NADPH-hemoprotein reductase] + O2 + a steroid = oxidized [NADPH-hemoprotein reductase] + H2O + H+ + 15alpha-hydroxy steroid.